{
  "gene_symbol": "CDIP1",
  "term_label": "zinc ion binding",
  "gene": "UniProtKB:Q9H305",
  "term_id": "GO:0008270",
  "gene_name": "Cell death-inducing p53-target protein 1"
}